{
  "gene_symbol": "LYNX1",
  "gene_name": "Ly-6_neurotoxin-like protein 1",
  "term_id": "GO:0095500",
  "term_label": "acetylcholine receptor signaling pathway",
  "gene": "UniProtKB:P0DP58"
}